{
  "term_id": "UNKNOWN:0001",
  "term_label": "Unknown molecular function",
  "gene_name": "MAP3K12-binding inhibitory protein 1",
  "gene": "UniProtKB:Q9NS73",
  "gene_symbol": "MBIP"
}